{
  "term_id": "UNKNOWN:0001",
  "gene_symbol": "GON7",
  "gene_name": "EKC_KEOPS complex subunit GON7",
  "term_label": "Unknown molecular function",
  "gene": "UniProtKB:Q9BXV9"
}